negative regulation of silent mating-type cassette heterochromatin formation [GO:0061186] (biological process) Definition: Any process that decreases the frequency, rate, or extent of heterochromatin formation at silent mating-type cassette. References: PMID:10388812 Sources: GOC:dph Also known as: negative regulation of chromatin silencing at silent mating-type cassette, negative regulation of silent mating-type cassette heterochromatin assembly Relationships: is a type of negative regulation of heterochromatin formation [GO:0031452]; is a type of regulation of silent mating-type cassette heterochromatin formation [GO:0090054]; negatively regulates silent mating-type cassette heterochromatin formation [GO:0030466]